protein secretion by the type III secretion system [GO:0030254] (biological process) Also known as: protein secretion by the T3S, protein secretion by the T3SS, protein secretion by the TTSS, protein secretion by the type III protein secretion system, type III protein secretion system Definition: The process in which proteins are transferred into the extracellular milieu or directly into host cells by the bacterial type III secretion system; secretion occurs in a continuous process without the distinct presence of periplasmic intermediates and does not involve proteolytic processing of secreted proteins. Sources: GOC:pamgo_curators Relationships: is a type of GO:0009306; is a type of protein transmembrane transport [GO:0071806] Note: Note that this term represents an activity and not a cellular structure. Consider also annotating to the cellular component term 'type III protein secretion system complex ; GO:0030257'. Note that this term is used for annotation of proteins that compose the secretion complex but not the proteins being secreted.